intracellular protein localization [GO:0008104] (biological process) Also known as: protein localization, cellular protein localisation, cellular protein localization, protein localisation, channel localizer activity, asymmetric protein localisation, asymmetric protein localization, establishment and maintenance of asymmetric protein localization, establishment and maintenance of protein localization Subtypes: GO:0007318, protein transport [GO:0015031], protein import into peroxisome matrix, docking [GO:0016560], protein localization to organelle [GO:0033365], protein localization to cell surface [GO:0034394], GO:0034497, protein localization to myelin sheath abaxonal region [GO:0035750], protein localization to trailing edge [GO:0036051], regulation of translation by machinery localization [GO:0043143], asymmetric protein localization involved in cell fate determination [GO:0045167], GO:0045175, apical protein localization [GO:0045176], protein localization involved in acrosome reaction [GO:0060476], GO:0061586, GO:0061938, protein localization to membrane [GO:0072657], protein localization to cell division site [GO:0072741], protein localization involved in establishment of planar polarity [GO:0090251], protein localization to bud neck [GO:0097271], GO:0099612, GO:1901703, GO:1902414, protein localization to cell leading edge [GO:1902463], protein localization to microvillus [GO:1904106], protein localization to cytosolic proteasome complex [GO:1904327], GO:1905719, GO:1990146, protein localization to cell tip [GO:1990151], protein localization to cell periphery [GO:1990778] Regulation: regulated by GO:0032880; negatively regulated by negative regulation of protein localization [GO:1903828]; positively regulated by positive regulation of protein localization [GO:1903829] Definition: Any process in which a protein is transported to, or maintained in, a specific location. Sources: GOC:ai Relationships: is a type of GO:0033036